{
  "gene_name": "Adenylate cyclase type 4",
  "term_id": "GO:0004016",
  "gene_symbol": "ADCY4",
  "gene": "UniProtKB:Q8NFM4",
  "term_label": "adenylate cyclase activity"
}